{
  "gene_name": "CRACD-like protein",
  "gene": "UniProtKB:Q6NV74",
  "gene_symbol": "CRACDL",
  "term_id": "UNKNOWN:0001",
  "term_label": "Unknown molecular function"
}